{
  "gene": "UniProtKB:O60806",
  "term_label": "chromatin",
  "term_id": "GO:0000785",
  "gene_name": "T-box transcription factor TBX19",
  "gene_symbol": "TBX19"
}